{
  "term_label": "protein serine/threonine kinase activity",
  "gene_name": "Serine_threonine-protein kinase LATS1",
  "term_id": "GO:0004674",
  "gene": "UniProtKB:O95835",
  "gene_symbol": "LATS1"
}